{
  "gene": "UniProtKB:A0A087WUV0",
  "term_label": "DNA-binding transcription factor activity, RNA polymerase II-specific",
  "term_id": "GO:0000981",
  "gene_name": "Zinc finger protein 892",
  "gene_symbol": "ZNF892"
}